albendazole monooxygenase activity [GO:0047638] (molecular function) Definition: Catalysis of the reaction: albendazole + H+ + NADPH + O2 = albendazole S-oxide + H2O + NADP+. Sources: EC:1.14.13.32, RHEA:10796 Relationships: is a type of oxidoreductase activity, acting on paired donors, with incorporation or reduction of molecular oxygen, NAD(P)H as one donor, and incorporation of one atom of oxygen [GO:0016709] Also known as: albendazole oxidase activity, albendazole sulfoxidase activity, albendazole,NADPH:oxygen oxidoreductase (sulfoxide-forming)